{
  "gene": "UniProtKB:O60774",
  "term_label": "taurine biosynthetic process",
  "term_id": "GO:0042412",
  "gene_symbol": "FMO6P",
  "gene_name": "Putative dimethylaniline monooxygenase [N-oxide-forming] 6"
}